{
  "gene_symbol": "CCL28",
  "gene_name": "C-C motif chemokine 28",
  "term_id": "GO:0008009",
  "term_label": "chemokine activity",
  "gene": "UniProtKB:Q9NRJ3"
}